{
  "gene_name": "Gamma-aminobutyric acid receptor subunit alpha-1",
  "term_label": "benzodiazepine receptor activity",
  "gene_symbol": "GABRA1",
  "gene": "UniProtKB:P14867",
  "term_id": "GO:0008503"
}